{
  "term_id": "GO:0005737",
  "gene_symbol": "SH2D4A",
  "gene_name": "SH2 domain-containing protein 4A",
  "term_label": "cytoplasm",
  "gene": "UniProtKB:Q9H788"
}